{
  "term_id": "GO:0050679",
  "gene_symbol": "ERBB2",
  "gene_name": "Receptor tyrosine-protein kinase erbB-2",
  "gene": "UniProtKB:P04626",
  "term_label": "positive regulation of epithelial cell proliferation"
}